{
  "gene": "UniProtKB:Q9BYX4",
  "gene_name": "Interferon-induced helicase C domain-containing protein 1",
  "gene_symbol": "IFIH1",
  "term_label": "double-stranded RNA binding",
  "term_id": "GO:0003725"
}